{
  "term_id": "UNKNOWN:0003",
  "gene": "UniProtKB:Q8IZS7",
  "gene_symbol": "CLECL1P",
  "term_label": "Unknown cellular component",
  "gene_name": "Putative C-type lectin-like domain family 1"
}